{
  "term_label": "G2/M transition of mitotic cell cycle",
  "gene_symbol": "CDK1",
  "gene": "UniProtKB:P06493",
  "gene_name": "Cyclin-dependent kinase 1",
  "term_id": "GO:0000086"
}